{
  "gene_name": "Homeobox protein Meis3",
  "term_label": "hemopoiesis",
  "term_id": "GO:0030097",
  "gene_symbol": "MEIS3",
  "gene": "UniProtKB:Q99687"
}